ascospore wall assembly [GO:0030476] (biological process) Relationships: is a type of developmental process involved in reproduction [GO:0003006]; is a type of spore wall assembly [GO:0042244]; is a type of GO:0071940; is_a meiotic cell cycle process [GO:1903046]; is part of ascospore wall biogenesis [GO:0070591] References: PMID:14702385 Sources: GOC:mcc Also known as: spore wall assembly Definition: The aggregation, arrangement and bonding together of a set of components to form an ascospore wall. During sporulation in Ascomycota, each ascospore nucleus becomes surrounded by a specialized spore wall, formed by deposition of spore wall components in the lumenal space between the outer and inner leaflets of the prospore membrane. An example of this process is found in Saccharomyces cerevisiae.